{
  "term_label": "RNA export from nucleus",
  "gene_symbol": "NPAP1",
  "term_id": "GO:0006405",
  "gene_name": "Nuclear pore-associated protein 1",
  "gene": "UniProtKB:Q9NZP6"
}